{
  "gene": "UniProtKB:A0M8Q6",
  "gene_name": "Immunoglobulin lambda constant 7",
  "gene_symbol": "IGLC7",
  "term_label": "IgG immunoglobulin complex",
  "term_id": "GO:0071735"
}